{
  "gene_symbol": "LCE3E",
  "gene_name": "Late cornified envelope protein 3E",
  "term_id": "UNKNOWN:0001",
  "term_label": "Unknown molecular function",
  "gene": "UniProtKB:Q5T5B0"
}